negative regulation of sister chromatid segregation [GO:0033046] (BP) Definition: Any process that stops, prevents, or reduces the frequency, rate or extent of sister chromatid segregation. Relationships: is a type of GO:0033045; is a type of negative regulation of chromosome segregation [GO:0051985]; is a type of negative regulation of chromosome organization [GO:2001251]; negatively regulates GO:0000819 Subtypes: negative regulation of mitotic sister chromatid segregation [GO:0033048] Sources: GOC:mah